{
  "gene_name": "Glucose-6-phosphatase catalytic subunit 1",
  "gene_symbol": "G6PC1",
  "gene": "UniProtKB:P35575",
  "term_id": "GO:0006094",
  "term_label": "gluconeogenesis"
}